{
  "gene": "UniProtKB:P51688",
  "term_label": "lysosome",
  "gene_symbol": "SGSH",
  "term_id": "GO:0005764",
  "gene_name": "N-sulphoglucosamine sulphohydrolase"
}